{
  "gene_symbol": "MMP14",
  "term_label": "zymogen activation",
  "gene": "UniProtKB:P50281",
  "term_id": "GO:0031638",
  "gene_name": "Matrix metalloproteinase-14"
}